{
  "term_label": "ossification",
  "gene": "UniProtKB:O75596",
  "gene_symbol": "CLEC3A",
  "term_id": "GO:0001503",
  "gene_name": "C-type lectin domain family 3 member A"
}